protein serine/threonine kinase activator activity [GO:0043539] (molecular function) Definition: Binds to and increases the activity of a protein serine/threonine kinase. Sources: GOC:go_curators Also known as: protein ser/thr kinase activator activity Relationships: is_a GO:0030295; RO_0002213 protein serine/threonine kinase activity [GO:0004674] Subtypes: eukaryotic elongation factor-2 kinase activator activity [GO:0042557], GO:0061575